{
  "gene_name": "Histone H2A type 1-A",
  "gene_symbol": "H2AC1",
  "gene": "UniProtKB:Q96QV6",
  "term_id": "GO:0005634",
  "term_label": "nucleus"
}